{
  "gene_name": "Putative uncharacterized protein C10orf88-like",
  "term_id": "UNKNOWN:0003",
  "term_label": "Unknown cellular component",
  "gene_symbol": "Q499Y3",
  "gene": "UniProtKB:Q499Y3"
}